{
  "term_id": "GO:0047372",
  "term_label": "monoacylglycerol lipase activity",
  "gene_symbol": "ABHD6",
  "gene_name": "Monoacylglycerol lipase ABHD6",
  "gene": "UniProtKB:Q9BV23"
}